{
  "gene_symbol": "ZDHHC6",
  "gene_name": "Palmitoyltransferase ZDHHC6",
  "term_id": "GO:0005783",
  "term_label": "endoplasmic reticulum",
  "gene": "UniProtKB:Q9H6R6"
}